{
  "term_id": "GO:0000978",
  "gene_name": "Zinc finger protein 260",
  "gene_symbol": "ZNF260",
  "term_label": "RNA polymerase II cis-regulatory region sequence-specific DNA binding",
  "gene": "UniProtKB:Q3ZCT1"
}